{
  "gene_name": "Homeobox protein DBX1",
  "gene": "UniProtKB:A6NMT0",
  "term_id": "GO:0006357",
  "term_label": "regulation of transcription by RNA polymerase II",
  "gene_symbol": "DBX1"
}